{
  "term_id": "UNKNOWN:0001",
  "gene_symbol": "PLAC9",
  "term_label": "Unknown molecular function",
  "gene": "UniProtKB:Q5JTB6",
  "gene_name": "Placenta-specific protein 9"
}